{
  "gene_symbol": "TAF1",
  "term_id": "GO:0017025",
  "gene": "UniProtKB:P21675",
  "term_label": "TBP-class protein binding",
  "gene_name": "Transcription initiation factor TFIID subunit 1"
}